{
  "term_label": "cadherin binding",
  "term_id": "GO:0045296",
  "gene": "UniProtKB:Q96JQ0",
  "gene_symbol": "DCHS1",
  "gene_name": "Protocadherin-16"
}